intermembrane phospholipid transfer [GO:0120010] (biological process) Relationships: is a type of phospholipid transport [GO:0015914]; is a type of GO:0120009 Definition: The transport of phospholipids between membranes in which a phospholipid molecule is transported through an aqueous phase from the outer leaflet of a donor membrane to the outer leaflet of an acceptor membrane. References: PMID:20823909, PMID:24220498, PMID:25797198 Sources: GOC:krc